{
  "term_id": "GO:0030334",
  "gene_name": "Fibroblast growth factor 6",
  "term_label": "regulation of cell migration",
  "gene_symbol": "FGF6",
  "gene": "UniProtKB:P10767"
}